{
  "gene": "UniProtKB:Q8NI35",
  "term_label": "bicellular tight junction",
  "term_id": "GO:0005923",
  "gene_name": "InaD-like protein",
  "gene_symbol": "PATJ"
}